extracellular isoamylase complex [GO:0010367] (cellular component) Definition: A protein complex whose composition varies amongst species; in rice it probably exists in a homo-tetramer to homo-hexamer form and in Gram negative bacteria as a dimer. Functions in the hydrolysis of alpha-(1,6)-D-glucosidic branch linkages. Isoamylases in animals are localized in the extracellular space. Sources: GOC:tair_curators Relationships: is a type of GO:0043033; BFO_0000050 extracellular region [GO:0005576]